interleukin-16 receptor activity [GO:0042012] (MF) Definition: Combining with interleukin-16 and transmitting the signal from one side of the membrane to the other to initiate a change in cell activity. Sources: GOC:jl, GOC:signaling Also known as: IL-16 receptor activity, IL-16R Relationships: is a type of cytokine receptor activity [GO:0004896]; has part interleukin-16 binding [GO:0042011]